{
  "gene_symbol": "ZFHX4",
  "gene_name": "Zinc finger homeobox protein 4",
  "term_id": "GO:0000978",
  "gene": "UniProtKB:Q86UP3",
  "term_label": "RNA polymerase II cis-regulatory region sequence-specific DNA binding"
}